gluconolactonase activity [GO:0004341] (MF) Sources: EC:3.1.1.17 Relationships: is a type of carboxylic ester hydrolase activity [GO:0052689] Also known as: lactonase activity, D-glucono-1,5-lactone lactonohydrolase activity, aldonolactonase activity, glucono-delta-lactonase activity, gulonolactonase activity Definition: Catalysis of the reaction: D-glucono-1,5-lactone + H2O = D-gluconate.